putrescine oxidase activity [GO:0050232] (molecular function) Definition: Catalysis of the reaction: H2O + O2 + putrescine = 4-aminobutanal + H2O2 + NH4+. Sources: RHEA:18273 Relationships: is a type of diamine oxidase activity [GO:0052597] Also known as: putrescine:oxygen oxidoreductase (deaminating)